{
  "term_id": "UNKNOWN:0002",
  "term_label": "Unknown biological process",
  "gene": "UniProtKB:A0A286YF58",
  "gene_symbol": "TMEM271",
  "gene_name": "Transmembrane protein 271"
}